{
  "term_id": "GO:0000977",
  "gene": "UniProtKB:Q96PT3",
  "term_label": "RNA polymerase II transcription regulatory region sequence-specific DNA binding",
  "gene_symbol": "DUX5",
  "gene_name": "Double homeobox protein 5"
}